{
  "gene_symbol": "CORO1A",
  "term_id": "GO:0005886",
  "gene": "UniProtKB:P31146",
  "term_label": "plasma membrane",
  "gene_name": "Coronin-1A"
}